{
  "term_label": "Unknown cellular component",
  "term_id": "UNKNOWN:0003",
  "gene_name": "Putative cTAGE family member 3",
  "gene": "UniProtKB:Q8IX95",
  "gene_symbol": "CTAGE3P"
}